{
  "term_id": "GO:0090249",
  "gene_name": "Serine_threonine-protein phosphatase 2A regulatory subunit B'' subunit alpha",
  "gene": "UniProtKB:Q06190",
  "gene_symbol": "PPP2R3A",
  "term_label": "regulation of cell migration involved in somitogenic axis elongation"
}